{
  "term_label": "sensory organ development",
  "gene_symbol": "ATOH7",
  "gene_name": "Transcription factor ATOH7",
  "gene": "UniProtKB:Q8N100",
  "term_id": "GO:0007423"
}